{
  "gene_name": "snRNA-activating protein complex subunit 3",
  "gene": "UniProtKB:Q92966",
  "gene_symbol": "SNAPC3",
  "term_label": "snRNA transcription by RNA polymerase II",
  "term_id": "GO:0042795"
}